{
  "gene_symbol": "NLRP6",
  "term_label": "acute inflammatory response",
  "gene": "UniProtKB:P59044",
  "gene_name": "NACHT, LRR and PYD domains-containing protein 6",
  "term_id": "GO:0002526"
}